{
  "gene_symbol": "HMCN2",
  "term_label": "axon",
  "gene": "UniProtKB:Q8NDA2",
  "gene_name": "Hemicentin-2",
  "term_id": "GO:0030424"
}